{
  "gene": "UniProtKB:O60895",
  "gene_name": "Receptor activity-modifying protein 2",
  "term_label": "G protein-coupled receptor signaling pathway",
  "term_id": "GO:0007186",
  "gene_symbol": "RAMP2"
}